{
  "gene_name": "B melanoma antigen 4",
  "term_id": "UNKNOWN:0002",
  "term_label": "Unknown biological process",
  "gene_symbol": "BAGE4",
  "gene": "UniProtKB:Q86Y28"
}